{
  "term_id": "GO:0005739",
  "gene_symbol": "COX5B",
  "gene_name": "Cytochrome c oxidase subunit 5B, mitochondrial",
  "term_label": "mitochondrion",
  "gene": "UniProtKB:P10606"
}